{
  "gene_name": "Melanoma-associated antigen B6B",
  "gene": "UniProtKB:A0A0J9YX57",
  "gene_symbol": "MAGEB6B",
  "term_id": "GO:0005634",
  "term_label": "nucleus"
}